{
  "term_id": "GO:0005886",
  "gene_name": "Tyrosine-protein kinase TXK",
  "term_label": "plasma membrane",
  "gene_symbol": "TXK",
  "gene": "UniProtKB:P42681"
}